{
  "gene_symbol": "LOXL4",
  "gene_name": "Lysyl oxidase homolog 4",
  "gene": "UniProtKB:Q96JB6",
  "term_label": "extracellular matrix",
  "term_id": "GO:0031012"
}